{
  "term_id": "UNKNOWN:0003",
  "term_label": "Unknown cellular component",
  "gene_name": "Serine_threonine-protein kinase Nek9",
  "gene_symbol": "NEK9",
  "gene": "UniProtKB:Q8TD19"
}